basal dendrite development [GO:0150018] (biological process) Relationships: is a type of dendrite development [GO:0016358] Definition: The process whose specific outcome is the progression of a basal dendrite over time, from its formation to the mature structure. References: PMID:22683681 Sources: GOC:aruk, GOC:bc